{
  "term_label": "Unknown biological process",
  "gene": "UniProtKB:Q8N4Y2",
  "gene_name": "EF-hand calcium-binding domain-containing protein 4A",
  "gene_symbol": "CRACR2B",
  "term_id": "UNKNOWN:0002"
}